{
  "term_label": "perinuclear region of cytoplasm",
  "gene_name": "Synaptojanin-1",
  "gene_symbol": "SYNJ1",
  "gene": "UniProtKB:O43426",
  "term_id": "GO:0048471"
}